{
  "term_id": "GO:0005634",
  "term_label": "nucleus",
  "gene": "UniProtKB:P0CW00",
  "gene_name": "Testis-specific Y-encoded protein 8",
  "gene_symbol": "TSPY8"
}